{
  "gene_symbol": "TMEM80",
  "term_label": "non-motile cilium assembly",
  "gene": "UniProtKB:Q96HE8",
  "gene_name": "Transmembrane protein 80",
  "term_id": "GO:1905515"
}